intracellular distribution of mitochondria [GO:0048312] (BP) Definition: Any process that establishes the spatial arrangement of mitochondria within the cell. Relationships: is a type of mitochondrion distribution [GO:0048311] Sources: GOC:jid Also known as: mitochondria positioning within cell, mitochondrion positioning within cell